{
  "term_label": "proteasome-mediated ubiquitin-dependent protein catabolic process",
  "gene_symbol": "PSMB10",
  "term_id": "GO:0043161",
  "gene_name": "Proteasome subunit beta type-10",
  "gene": "UniProtKB:P40306"
}